{
  "gene": "UniProtKB:Q9UQ16",
  "gene_name": "Dynamin-3",
  "term_id": "GO:0003924",
  "term_label": "GTPase activity",
  "gene_symbol": "DNM3"
}